{
  "gene_name": "Uncharacterized protein C11orf42",
  "gene": "UniProtKB:Q8N5U0",
  "term_id": "UNKNOWN:0001",
  "gene_symbol": "C11orf42",
  "term_label": "Unknown molecular function"
}